{
  "gene_symbol": "RPS10",
  "gene_name": "Small ribosomal subunit protein eS10",
  "gene": "UniProtKB:P46783",
  "term_label": "structural constituent of ribosome",
  "term_id": "GO:0003735"
}